{
  "term_id": "GO:0003723",
  "gene_name": "RNA-binding protein 26",
  "gene": "UniProtKB:Q5T8P6",
  "term_label": "RNA binding",
  "gene_symbol": "RBM26"
}